regulation of T-helper 17 cell lineage commitment [GO:2000328] (biological process) Definition: Any process that modulates the frequency, rate or extent of T-helper 17 cell lineage commitment. Also known as: regulation of T-helper 17 cell fate commitment, regulation of Th17 cell lineage commitment, regulation of Th17 fate commitment Subtypes: negative regulation of T-helper 17 cell lineage commitment [GO:2000329], positive regulation of T-helper 17 cell lineage commitment [GO:2000330] Relationships: is_a GO:0010453; is a type of regulation of T-helper 17 cell differentiation [GO:2000319]; regulates T-helper 17 cell lineage commitment [GO:0072540] Sources: GOC:BHF, GOC:mah